{
  "term_id": "UNKNOWN:0001",
  "gene_name": "Endogenous retrovirus group V member 2 Env polyprotein",
  "term_label": "Unknown molecular function",
  "gene_symbol": "ERVV-2",
  "gene": "UniProtKB:B6SEH9"
}